{
  "gene": "UniProtKB:Q75WM6",
  "gene_symbol": "H1-7",
  "term_label": "nucleosomal DNA binding",
  "gene_name": "Testis-specific H1 histone",
  "term_id": "GO:0031492"
}